{
  "term_label": "adaptive thermogenesis",
  "gene_symbol": "UCP1",
  "gene": "UniProtKB:P25874",
  "term_id": "GO:1990845",
  "gene_name": "Mitochondrial brown fat uncoupling protein 1"
}